cell motility involved in camera-type eye morphogenesis [GO:0003411] (biological process) Definition: Any process involved in the controlled self-propelled movement of a cell that results in translocation of the cell from one place to another and contributes to the physical shaping or formation of the camera-type eye. Sources: GOC:ascb_2009, GOC:dph, GOC:tb Relationships: is a type of cell motility [GO:0048870]; is part of camera-type eye morphogenesis [GO:0048593]